{
  "gene_symbol": "SHH",
  "gene_name": "Sonic hedgehog protein",
  "term_id": "GO:0007224",
  "term_label": "smoothened signaling pathway",
  "gene": "UniProtKB:Q15465"
}